acyloxyacyl hydrolase activity [GO:0050528] (molecular function) Relationships: is a type of carboxylic ester hydrolase activity [GO:0052689] Sources: EC:3.1.1.77, MetaCyc:3.1.1.77-RXN Definition: Catalysis of the reaction: 3-(acyloxy)acyl group of bacterial toxin = 3-hydroxyacyl group of bacterial toxin + a fatty acid.